{
  "term_label": "cytosol",
  "gene_name": "Folliculin",
  "term_id": "GO:0005829",
  "gene_symbol": "FLCN",
  "gene": "UniProtKB:Q8NFG4"
}